{
  "gene_symbol": "LRBA",
  "term_id": "GO:0000423",
  "gene": "UniProtKB:P50851",
  "term_label": "mitophagy",
  "gene_name": "Lipopolysaccharide-responsive and beige-like anchor protein"
}